{
  "term_id": "GO:0035861",
  "term_label": "site of double-strand break",
  "gene": "UniProtKB:Q9Y253",
  "gene_name": "DNA polymerase eta",
  "gene_symbol": "POLH"
}